{
  "gene_symbol": "HEXA-AS1",
  "term_id": "UNKNOWN:0002",
  "gene": "UniProtKB:Q9H8Q6",
  "term_label": "Unknown biological process",
  "gene_name": "Putative uncharacterized protein encoded by HEXA-AS1"
}